{
  "gene": "UniProtKB:Q8TDU9",
  "term_label": "plasma membrane",
  "gene_name": "Relaxin-3 receptor 2",
  "term_id": "GO:0005886",
  "gene_symbol": "RXFP4"
}